negative regulation of cell-cell adhesion mediated by cadherin [GO:2000048] (biological process) Relationships: is a type of negative regulation of cell-cell adhesion [GO:0022408]; is_a GO:2000047; negatively regulates cell-cell adhesion mediated by cadherin [GO:0044331] Sources: GOC:obol Definition: Any process that stops, prevents, or reduces the frequency, rate or extent of cell-cell adhesion mediated by cadherin.